phosphopantothenoylcysteine decarboxylase activity [GO:0004633] (molecular function) Definition: Catalysis of the reaction: N-[(R)-4-phosphonatopantothenoyl]-L-cysteinate + H+ = CO2 + pantetheine 4'-phosphate. Also known as: 4-phosphopantothenoyl-L-cysteine decarboxylase activity, 4-phosphopantotheoylcysteine decarboxylase activity, N-((R)-4'-phosphopantothenoyl)-L-cysteine carboxy-lyase activity, N-[(R)-4'-phosphopantothenoyl]-L-cysteine carboxy-lyase (pantotheine-4'-phosphate-forming), N-[(R)-4'-phosphopantothenoyl]-L-cysteine carboxy-lyase activity, PPC-decarboxylase activity Sources: EC:4.1.1.36, RHEA:16793 Relationships: is a type of GO:0016831